{
  "gene_symbol": "TMEM199",
  "gene_name": "Transmembrane protein 199",
  "term_label": "Unknown molecular function",
  "term_id": "UNKNOWN:0001",
  "gene": "UniProtKB:Q8N511"
}